capsorubin catabolic process [GO:1901865] (biological process) Definition: The chemical reactions and pathways resulting in the breakdown of capsorubin. Sources: GOC:TermGenie, GOC:yaf, UniPathway:UPA00807 Also known as: capsorubin breakdown, capsorubin catabolism, capsorubin degradation Relationships: is a type of xanthophyll catabolic process [GO:0016124]